{
  "term_label": "cytoplasm",
  "gene_name": "14-3-3 protein epsilon",
  "gene_symbol": "YWHAE",
  "term_id": "GO:0005737",
  "gene": "UniProtKB:P62258"
}